phosphinothricin biosynthetic process [GO:1901766] (biological process) Also known as: phosphinothricin anabolism, phosphinothricin biosynthesis, phosphinothricin formation, phosphinothricin synthesis Sources: GOC:TermGenie, GOC:yaf, UniPathway:UPA00168 Relationships: is a type of biosynthetic process [GO:0009058]; is a type of GO:1901764 Definition: The chemical reactions and pathways resulting in the formation of phosphinothricin.